fructose 1,6-bisphosphate 1-phosphatase activity [GO:0042132] (molecular function) Definition: Catalysis of the reaction: D-fructose 1,6-bisphosphate + H2O = D-fructose 6-phosphate + phosphate. Sources: EC:3.1.3.11 Also known as: fructose-bisphosphatase activity, hexosediphosphatase activity, D-fructose 1,6-diphosphatase activity, D-fructose-1,6-bisphosphate 1-phosphohydrolase activity, D-fructose-1,6-bisphosphate phosphatase activity, FBPase activity, fructose 1,6-bisphosphatase activity, fructose 1,6-bisphosphate phosphatase activity, fructose 1,6-diphosphatase activity, fructose 1,6-diphosphate phosphatase activity, fructose bisphosphate phosphatase activity, fructose diphosphatase activity, fructose diphosphate phosphatase activity, fructose-1,6-bisphosphatase activity, hexose bisphosphatase activity, hexose diphosphatase activity Relationships: is a type of sugar-phosphatase activity [GO:0050308]